{
  "gene_symbol": "MFSD12",
  "gene_name": "Major facilitator superfamily domain-containing protein 12",
  "term_id": "GO:0005886",
  "gene": "UniProtKB:Q6NUT3",
  "term_label": "plasma membrane"
}